{
  "term_id": "GO:0004601",
  "gene": "UniProtKB:Q96SL4",
  "gene_name": "Glutathione peroxidase 7",
  "gene_symbol": "GPX7",
  "term_label": "peroxidase activity"
}